sperm migration through the uterotubal junction [GO:0160131] (biological process) Definition: The controlled self-propelled movement of a sperm cell from the uterus through the uterotubal junction (UTJ) into the oviduct, where interaction between the sperm and the UTJ acts as a major selective barrier for sperm, allowing only living, motile, uncapacitated, morphologically normal sperm with intact acrosomes to pass from the uterus into the oviduct. Relationships: is a type of cell migration [GO:0016477]; is part of multicellular organismal reproductive process [GO:0048609]; has part flagellated sperm motility [GO:0030317] References: PMID:29353867, PMID:31131960, PMID:32712384, PMID:34057175 Sources: GOC:krc Also known as: sperm migration from the uterus to the oviduct, sperm migration through the UTJ